{
  "gene_name": "Beta-defensin 113",
  "term_label": "Unknown cellular component",
  "gene_symbol": "DEFB113",
  "gene": "UniProtKB:Q30KQ7",
  "term_id": "UNKNOWN:0003"
}